{
  "gene": "UniProtKB:O14713",
  "term_label": "negative regulation of substrate adhesion-dependent cell spreading",
  "gene_symbol": "ITGB1BP1",
  "gene_name": "Integrin beta-1-binding protein 1",
  "term_id": "GO:1900025"
}